extrathymic T cell differentiation [GO:0033078] (biological process) Sources: GOC:add, ISBN:0781735149 Definition: The process in which a precursor cell type acquires the specialized features of a T cell via a differentiation pathway independent of the thymus. Also known as: extrathymic T cell development Relationships: is a type of GO:0030217 Regulation: regulated by regulation of extrathymic T cell differentiation [GO:0033082]; negatively regulated by negative regulation of extrathymic T cell differentiation [GO:0033086]; positively regulated by positive regulation of extrathymic T cell differentiation [GO:0033090] Note: Note that immunologists typically use the word 'development' to refer to cells of B or T cell lineages undergoing the process that GO describes as 'cell differentiation'.